{
  "gene_name": "Taste receptor type 1 member 3",
  "term_id": "GO:0050917",
  "gene_symbol": "TAS1R3",
  "term_label": "sensory perception of umami taste",
  "gene": "UniProtKB:Q7RTX0"
}